{
  "gene_name": "Inward rectifier potassium channel 13",
  "gene": "UniProtKB:O60928",
  "term_label": "potassium ion import across plasma membrane",
  "term_id": "GO:1990573",
  "gene_symbol": "KCNJ13"
}